triphosphoric monoester hydrolase activity [GO:0016793] (molecular function) Relationships: is a type of phosphoric ester hydrolase activity [GO:0042578] Subtypes: dGTPase activity [GO:0008832], deoxynucleoside triphosphate hydrolase activity [GO:0106375] Definition: Catalysis of the hydrolysis of a triphosphoester to give a triphosphate group and a free hydroxyl group. Sources: EC:3.1.5.-